{
  "gene_name": "Mitogen-activated protein kinase kinase kinase 4",
  "term_id": "GO:0038066",
  "gene_symbol": "MAP3K4",
  "gene": "UniProtKB:Q9Y6R4",
  "term_label": "p38MAPK cascade"
}